{
  "gene_symbol": "IL18R1",
  "term_label": "interleukin-18-mediated signaling pathway",
  "term_id": "GO:0035655",
  "gene": "UniProtKB:Q13478",
  "gene_name": "Interleukin-18 receptor 1"
}